{
  "term_label": "RNA polymerase II cis-regulatory region sequence-specific DNA binding",
  "gene_name": "T-box transcription factor TBX21",
  "gene": "UniProtKB:Q9UL17",
  "term_id": "GO:0000978",
  "gene_symbol": "TBX21"
}